mesonephric interstitial fibroblast differentiation [GO:0061266] (biological process) Definition: The process in which relatively unspecialized cells acquire specialized structural and/or functional features that characterize the interstitial fibroblasts of the mesonephros as it progresses from its formation to the mature state. Sources: GOC:mtg_kidney_jan10 Also known as: mesonephros interstitial cell differentiation Relationships: is a type of GO:0061208; is a type of kidney interstitial fibroblast differentiation [GO:0072071]